sulfurtransferase complex [GO:1990228] (cellular component) Definition: A protein complex capable of catalyzing the transfer of sulfur atoms from one compound (donor) to another (acceptor). Relationships: is a type of transferase complex [GO:1990234]; is part of cytosol [GO:0005829] Subtypes: cytosolic tRNA wobble base thiouridylase complex [GO:0002144], thiazole synthase complex [GO:1902507], molybdopterin synthase complex [GO:1990140], L-cysteine desulfurase complex [GO:1990221] Also known as: sulfur transfer complex, SufE complex, SufE dimer, ThiF-ThiS complex References: PMID:17350958 Sources: GOC:bhm